{
  "term_label": "NAD(P)HX epimerase activity",
  "gene_name": "YjeF N-terminal domain-containing protein 3",
  "term_id": "GO:0052856",
  "gene_symbol": "YJEFN3",
  "gene": "UniProtKB:A6XGL0"
}